regulation of polysaccharide metabolic process [GO:0032881] (BP) Definition: Any process that modulates the frequency, rate or extent of the chemical reactions and pathways involving polysaccharides. Relationships: is a type of regulation of carbohydrate metabolic process [GO:0006109]; is a type of regulation of macromolecule metabolic process [GO:0060255]; regulates polysaccharide metabolic process [GO:0005976] Sources: GOC:mah Subtypes: GO:0032882, regulation of polysaccharide biosynthetic process [GO:0032885], regulation of alpha-glucan metabolic process [GO:0032948], regulation of beta-glucan metabolic process [GO:0032950], regulation of glycogen metabolic process [GO:0070873], regulation of cell wall pectin metabolic process [GO:1902066], regulation of glucomannan catabolic process [GO:2000898], regulation of starch metabolic process [GO:2000904], regulation of galactoglucomannan catabolic process [GO:2000912], regulation of cellodextrin catabolic process [GO:2000927], GO:2000957, GO:2000966, GO:2000988, regulation of galactomannan catabolic process [GO:2000991], regulation of pectin catabolic process [GO:2001003]